{
  "gene_symbol": "OR11L1",
  "gene_name": "Olfactory receptor 11L1",
  "gene": "UniProtKB:Q8NGX0",
  "term_id": "UNKNOWN:0002",
  "term_label": "Unknown biological process"
}